{
  "gene_name": "Small cysteine and glycine repeat-containing protein 1",
  "term_id": "UNKNOWN:0002",
  "gene_symbol": "SCYGR1",
  "term_label": "Unknown biological process",
  "gene": "UniProtKB:A0A286YEY9"
}